{
  "term_label": "Unknown cellular component",
  "gene_symbol": "KDM2A",
  "gene_name": "Lysine-specific demethylase 2A",
  "term_id": "UNKNOWN:0003",
  "gene": "UniProtKB:Q9Y2K7"
}